{
  "term_label": "positive regulation of cell population proliferation",
  "gene": "UniProtKB:Q8NI17",
  "term_id": "GO:0008284",
  "gene_symbol": "IL31RA",
  "gene_name": "Interleukin-31 receptor subunit alpha"
}